{
  "gene_symbol": "RPL39",
  "gene_name": "Large ribosomal subunit protein eL39",
  "term_id": "GO:0002181",
  "term_label": "cytoplasmic translation",
  "gene": "UniProtKB:P62891"
}